{
  "gene_name": "Cysteine and tyrosine-rich protein 1",
  "gene_symbol": "CYYR1",
  "gene": "UniProtKB:Q96J86",
  "term_id": "UNKNOWN:0003",
  "term_label": "Unknown cellular component"
}